{
  "gene_symbol": "CNKSR2",
  "term_label": "protein-macromolecule adaptor activity",
  "term_id": "GO:0030674",
  "gene_name": "Connector enhancer of kinase suppressor of ras 2",
  "gene": "UniProtKB:Q8WXI2"
}